{
  "gene": "UniProtKB:Q5XG99",
  "gene_symbol": "LYSMD4",
  "term_id": "UNKNOWN:0002",
  "term_label": "Unknown biological process",
  "gene_name": "LysM and putative peptidoglycan-binding domain-containing protein 4"
}